{
  "term_id": "GO:0031297",
  "gene_name": "Probable crossover junction endonuclease EME2",
  "gene": "UniProtKB:A4GXA9",
  "gene_symbol": "EME2",
  "term_label": "replication fork processing"
}